regulation of thymine transport [GO:0035365] (biological process) Also known as: regulation of 5-methyluracil transport Subtypes: negative regulation of thymine transport [GO:0035366], positive regulation of thymine transport [GO:0035367] Relationships: is a type of regulation of nucleobase-containing compound transport [GO:0032239]; regulates thymine transport [GO:0035364] Definition: Any process that modulates the frequency, rate or extent of the directed movement of thymine, 5-methyluracil, into, out of or within a cell, or between cells, by means of some agent such as a transporter or pore. Sources: GOC:bf, GOC:sl